{
  "term_label": "ciliary transition zone",
  "gene_symbol": "CIBAR2",
  "gene_name": "CBY1-interacting BAR domain-containing protein 2",
  "term_id": "GO:0035869",
  "gene": "UniProtKB:Q6ZTR7"
}